{
  "gene_symbol": "CFB",
  "term_label": "Unknown cellular component",
  "gene": "UniProtKB:P00751",
  "gene_name": "Complement factor B",
  "term_id": "UNKNOWN:0003"
}